{
  "gene_name": "Zinc finger and BTB domain-containing protein 26",
  "gene": "UniProtKB:Q9HCK0",
  "gene_symbol": "ZBTB26",
  "term_label": "nucleoplasm",
  "term_id": "GO:0005654"
}